{
  "term_label": "RNA polymerase II general transcription initiation factor activity",
  "gene_symbol": "TAF11",
  "term_id": "GO:0016251",
  "gene_name": "Transcription initiation factor TFIID subunit 11",
  "gene": "UniProtKB:Q15544"
}